{
  "gene_symbol": "ATRX",
  "gene": "UniProtKB:P46100",
  "gene_name": "Transcriptional regulator ATRX",
  "term_label": "nucleus",
  "term_id": "GO:0005634"
}